{
  "term_id": "UNKNOWN:0002",
  "term_label": "Unknown biological process",
  "gene_symbol": "HDDC2",
  "gene": "UniProtKB:Q7Z4H3",
  "gene_name": "5'-deoxynucleotidase HDDC2"
}